negative regulation of isotype switching to IgE isotypes [GO:0048294] (biological process) Relationships: is_a negative regulation of isotype switching [GO:0045829]; is a type of GO:0048293; negatively regulates GO:0048289 Sources: GOC:jid Also known as: down regulation of isotype switching to IgE isotypes, down-regulation of isotype switching to IgE isotypes, downregulation of isotype switching to IgE isotypes, negative regulation of class switch recombination to IgE isotypes, negative regulation of class switching to IgE isotypes, negative regulation of isotype switch recombination to IgE isotypes, inhibition of isotype switching to IgE isotypes Definition: Any process that stops, prevents, or reduces the frequency, rate or extent of isotype switching to IgE isotypes.